CST complex [GO:1990879] (cellular component) Relationships: is a type of nuclear telomere cap complex [GO:0000783] References: PMID:19854130, PMID:22965356 Sources: GOC:BHF, GOC:BHF_telomere, GOC:nc Definition: A complex formed by the association of Cdc13 (CTC1 in mammals) with Stn1 in yeast (OBFC1 in mammals) and Ten1 protein (also TEN1 in mammals) with single-stranded telomeric DNA. The CST complex plays a role in telomere protection. Also known as: CTC1-OBFC1-TEN1 complex, Cdc13-Stn1-Ten1 complex